{
  "gene_name": "Zinc finger protein 202",
  "term_id": "GO:0000978",
  "gene": "UniProtKB:O95125",
  "term_label": "RNA polymerase II cis-regulatory region sequence-specific DNA binding",
  "gene_symbol": "ZNF202"
}